{
  "gene_symbol": "DCUN1D3",
  "gene_name": "DCN1-like protein 3",
  "term_label": "protein neddylation",
  "gene": "UniProtKB:Q8IWE4",
  "term_id": "GO:0045116"
}